regulation of systemic arterial blood pressure by aortic arch baroreceptor feedback [GO:0003026] (biological process) Definition: The process that modulates blood pressure by sensing the amount of stretch occurring in the aorta and responding to the input via central nervous system control. Sources: GOC:dph, GOC:mtg_cardio, GOC:tb Relationships: is a type of nervous system process involved in regulation of systemic arterial blood pressure [GO:0001976]; is part of GO:0003025 Also known as: aortic arch baroreceptor control of systemic arterial blood pressure